extrinsic component of stromal side of plastid thylakoid membrane [GO:0035451] (CC) Relationships: is a type of GO:0035449; is part of stromal side of plastid thylakoid membrane [GO:0098572] Sources: GOC:bf, GOC:dos Definition: The component of a plastid thylakoid membrane consisting of gene products and protein complexes that are loosely bound to its stromal surface, but not integrated into the hydrophobic region. Also known as: extrinsic to stromal leaflet of plastid thylakoid membrane, peripheral to stromal side of plastid thylakoid membrane, extrinsic to stromal side of plastid thylakoid membrane